{
  "gene": "UniProtKB:P29377",
  "term_id": "GO:0048306",
  "gene_name": "Protein S100-G",
  "gene_symbol": "S100G",
  "term_label": "calcium-dependent protein binding"
}